cell projection assembly [GO:0030031] (biological process) Definition: Formation of a prolongation or process extending from a cell, e.g. a flagellum or axon. Relationships: is a type of GO:0022607; is a type of cell projection organization [GO:0030030] Subtypes: GO:0009297, bacterial-type flagellum assembly [GO:0044780], plasma membrane bounded cell projection assembly [GO:0120031], trichome papilla formation [GO:1905499] Also known as: formation of a cell surface projection, cell projection biogenesis Regulation: regulated by regulation of cell projection assembly [GO:0060491] References: PMID:18391171 Sources: GOC:jl, GOC:mah